{
  "gene_name": "Nociceptin receptor",
  "gene": "UniProtKB:P41146",
  "gene_symbol": "OPRL1",
  "term_label": "neuron projection",
  "term_id": "GO:0043005"
}